{
  "gene": "UniProtKB:P57075",
  "gene_symbol": "UBASH3A",
  "term_label": "Unknown molecular function",
  "term_id": "UNKNOWN:0001",
  "gene_name": "Ubiquitin-associated and SH3 domain-containing protein A"
}